{
  "gene_symbol": "HELZ2",
  "term_id": "GO:0003723",
  "gene_name": "Helicase with zinc finger domain 2",
  "gene": "UniProtKB:Q9BYK8",
  "term_label": "RNA binding"
}